{
  "gene_symbol": "FHIP1B",
  "gene": "UniProtKB:Q8N612",
  "term_id": "GO:0007040",
  "gene_name": "FHF complex subunit HOOK-interacting protein 1B",
  "term_label": "lysosome organization"
}